{
  "gene": "UniProtKB:Q9Y2I7",
  "term_id": "GO:0012506",
  "term_label": "vesicle membrane",
  "gene_name": "1-phosphatidylinositol 3-phosphate 5-kinase",
  "gene_symbol": "PIKFYVE"
}